{
  "gene_name": "Small ribosomal subunit protein mS23",
  "term_label": "Unknown biological process",
  "gene": "UniProtKB:Q9Y3D9",
  "term_id": "UNKNOWN:0002",
  "gene_symbol": "MRPS23"
}